{
  "gene_symbol": "MEIS3P2",
  "term_label": "animal organ morphogenesis",
  "term_id": "GO:0009887",
  "gene_name": "Putative homeobox protein Meis3-like 2",
  "gene": "UniProtKB:A8K0S8"
}